nuclear-transcribed mRNA poly(A) tail shortening [GO:0000289] (biological process) Sources: GOC:krc Also known as: 3' to 5' mRNA deadenylation, mRNA deadenylation, nuclear mRNA poly(A) tail shortening Definition: Shortening of the poly(A) tail of a nuclear-transcribed mRNA from full length to an oligo(A) length. Relationships: is a type of nuclear-transcribed mRNA catabolic process [GO:0000956]; is part of GO:0000288 Regulation: RO_0002211 by regulation of nuclear-transcribed mRNA poly(A) tail shortening [GO:0060211]; negatively regulated by negative regulation of nuclear-transcribed mRNA poly(A) tail shortening [GO:0060212]; positively regulated by positive regulation of nuclear-transcribed mRNA poly(A) tail shortening [GO:0060213]